GARP complex binding [GO:0062069] (MF) Definition: Binding to a GARP complex. Relationships: is a type of protein-containing complex binding [GO:0044877] References: PMID:20163565